{
  "gene": "UniProtKB:P08758",
  "term_label": "cytoplasm",
  "gene_name": "Annexin A5",
  "term_id": "GO:0005737",
  "gene_symbol": "ANXA5"
}